{
  "gene_symbol": "KRT73",
  "gene_name": "Keratin, type II cytoskeletal 73",
  "term_id": "GO:0030280",
  "gene": "UniProtKB:Q86Y46",
  "term_label": "structural constituent of skin epidermis"
}